{
  "gene_name": "Biotin--protein ligase",
  "gene": "UniProtKB:P50747",
  "gene_symbol": "HLCS",
  "term_id": "UNKNOWN:0002",
  "term_label": "Unknown biological process"
}